{
  "term_label": "Unknown cellular component",
  "gene_symbol": "PGPEP1",
  "gene": "UniProtKB:Q9NXJ5",
  "gene_name": "Pyroglutamyl-peptidase 1",
  "term_id": "UNKNOWN:0003"
}